positive regulation of polarized epithelial cell differentiation [GO:0030862] (BP) Definition: Any process that activates or increases the rate or extent of polarized epithelial cell differentiation. Sources: GOC:mah Relationships: is a type of positive regulation of epithelial cell differentiation [GO:0030858]; is a type of regulation of polarized epithelial cell differentiation [GO:0030860]; positively regulates polarized epithelial cell differentiation [GO:0030859] Also known as: up regulation of polarized epithelial cell differentiation, up-regulation of polarized epithelial cell differentiation, upregulation of polarized epithelial cell differentiation, activation of polarized epithelial cell differentiation, stimulation of polarized epithelial cell differentiation